{
  "term_id": "UNKNOWN:0001",
  "gene_name": "CUE domain-containing protein 1",
  "gene_symbol": "CUEDC1",
  "gene": "UniProtKB:Q9NWM3",
  "term_label": "Unknown molecular function"
}